anterior compartment pattern formation [GO:0007387] (biological process) Relationships: is a type of GO:0007386 Definition: The process giving rise to specification of cell identity in the anterior compartments of the segmented embryo. Sources: ISBN:0879694238, http://fly.ebi.ac.uk/allied-data/lk/interactive-fly/aimain/1aahome.htm Also known as: anterior compartment pattern specification